4-vinylphenol methyltransferase activity [GO:0160304] (molecular function) Relationships: is a type of O-methyltransferase activity [GO:0008171]; is_a GO:0008757 References: PMID:40562929 Definition: Catalysis of the reaction: 4-vinylphenol + S-adenosyl-L-methionine = 4-vinylanisole + S-adenosyl-L-homocysteine + H+.